{
  "term_label": "endoplasmic reticulum exit site",
  "term_id": "GO:0070971",
  "gene": "UniProtKB:Q8IX94",
  "gene_name": "cTAGE family member 4",
  "gene_symbol": "CTAGE4"
}